{
  "gene": "UniProtKB:A2A368",
  "gene_symbol": "MAGEB16",
  "gene_name": "Melanoma-associated antigen B16",
  "term_id": "UNKNOWN:0001",
  "term_label": "Unknown molecular function"
}